{
  "gene_symbol": "HTATSF1",
  "term_label": "RNA binding",
  "gene_name": "HIV Tat-specific factor 1",
  "term_id": "GO:0003723",
  "gene": "UniProtKB:O43719"
}